{
  "term_label": "extracellular space",
  "gene_symbol": "ADM2",
  "gene": "UniProtKB:Q7Z4H4",
  "term_id": "GO:0005615",
  "gene_name": "Protein ADM2"
}